{
  "gene_name": "Ezrin",
  "term_id": "GO:0005902",
  "term_label": "microvillus",
  "gene_symbol": "EZR",
  "gene": "UniProtKB:P15311"
}